positive regulation of macrophage fusion [GO:0034241] (biological process) Sources: GOC:mah Definition: Any process that activates or increases the frequency, rate or extent of macrophage fusion. Relationships: is a type of regulation of macrophage fusion [GO:0034239]; is a type of positive regulation of syncytium formation by plasma membrane fusion [GO:0060143]; positively regulates GO:0034238